{
  "gene_name": "Protein Wnt-8b",
  "term_id": "GO:0060070",
  "gene_symbol": "WNT8B",
  "term_label": "canonical Wnt signaling pathway",
  "gene": "UniProtKB:Q93098"
}